{
  "gene_symbol": "TLK2",
  "gene_name": "Serine_threonine-protein kinase tousled-like 2",
  "gene": "UniProtKB:Q86UE8",
  "term_id": "GO:0004674",
  "term_label": "protein serine/threonine kinase activity"
}